{
  "gene": "UniProtKB:O00445",
  "gene_name": "Synaptotagmin-5",
  "term_label": "calcium ion sensor activity",
  "term_id": "GO:0061891",
  "gene_symbol": "SYT5"
}